{
  "gene_name": "Protein arginine N-methyltransferase 2",
  "gene": "UniProtKB:P55345",
  "term_id": "GO:0005634",
  "gene_symbol": "PRMT2",
  "term_label": "nucleus"
}